2-heptyl-3-hydroxy-4(1H)-quinolone synthase activity [GO:0102164] (molecular function) Sources: EC:1.14.13.182, GOC:pz Relationships: is a type of oxidoreductase activity, acting on paired donors, with incorporation or reduction of molecular oxygen, NAD(P)H as one donor, and incorporation of one atom of oxygen [GO:0016709] Definition: Catalysis of the reaction: 2-heptyl-4-quinolone + NADH + O2 + H+ = 2-heptyl-3-hydroxy-4-quinolone + NAD + H2O.